{
  "gene_symbol": "GOLPH3L",
  "term_id": "GO:0007030",
  "term_label": "Golgi organization",
  "gene_name": "Golgi phosphoprotein 3-like",
  "gene": "UniProtKB:Q9H4A5"
}